{
  "term_id": "UNKNOWN:0001",
  "gene_name": "Ceroid-lipofuscinosis neuronal protein 6",
  "term_label": "Unknown molecular function",
  "gene_symbol": "CLN6",
  "gene": "UniProtKB:Q9NWW5"
}